{
  "term_label": "cytoplasm",
  "gene_name": "Kinesin-like protein KIF25",
  "gene_symbol": "KIF25",
  "gene": "UniProtKB:Q9UIL4",
  "term_id": "GO:0005737"
}